mitotic spindle pole body [GO:0044732] (cellular component) Relationships: is a type of spindle pole body [GO:0005816] Definition: The microtubule organizing center that forms as part of the mitotic cell cycle; functionally homologous to the animal cell centrosome. Sources: GOC:mah, GOC:vw Subtypes: old mitotic spindle pole body [GO:0071957], new mitotic spindle pole body [GO:0071958]